{
  "gene_name": "Metabotropic glutamate receptor 2",
  "term_id": "GO:0005886",
  "term_label": "plasma membrane",
  "gene": "UniProtKB:Q14416",
  "gene_symbol": "GRM2"
}